{
  "gene": "UniProtKB:O60610",
  "gene_name": "Protein diaphanous homolog 1",
  "term_id": "UNKNOWN:0001",
  "gene_symbol": "DIAPH1",
  "term_label": "Unknown molecular function"
}